amphiregulin production [GO:0140730] (biological process) Definition: The appearance of amphiregulin due to biosynthesis or secretion following a cellular stimulus, resulting in an increase in its intracellular or extracellular levels. Amphiregulin (AREG) is a ligand of the epidermal growth factor receptor (EGFR), a widely expressed transmembrane tyrosine kinase. AREG is synthesized as a membrane-anchored precursor protein that can engage in juxtacrine signaling on adjacent cells. Alternatively, after proteolytic processing by cell membrane proteases, mainly TACE/ADAM17, AREG is secreted and behaves as an autocrine or paracrine factor. Note: Note that this term is in the subset of terms that should not be used for direct gene product annotation. Instead, select one of the 'regulation' children terms. References: PMID:24463227 Regulation: regulated by GO:0140731; RO_0002213 by positive regulation of amphiregulin production [GO:0140732] Also known as: AREG production Relationships: is a type of cytokine production [GO:0001816]